tyrosine sensor activity [GO:0120285] (molecular function) Also known as: tyrosine sensing activity Relationships: is a type of amino acid sensor activity [GO:0140785]; has part L-tyrosine binding [GO:0072545] References: PMID:31498992 Sources: GOC:krc Definition: Binding to and responding, e.g. by conformational change, to changes in the cellular level of tyrosine.